{
  "gene_symbol": "NEIL1",
  "gene": "UniProtKB:Q96FI4",
  "gene_name": "Endonuclease 8-like 1",
  "term_id": "GO:0006284",
  "term_label": "base-excision repair"
}